{
  "term_label": "Unknown molecular function",
  "gene": "UniProtKB:Q6ZRC1",
  "term_id": "UNKNOWN:0001",
  "gene_symbol": "C4orf50",
  "gene_name": "Uncharacterized protein C4orf50"
}